{
  "gene_name": "Membrane protein MLC1",
  "gene_symbol": "MLC1",
  "gene": "UniProtKB:Q15049",
  "term_label": "cytoplasmic vesicle",
  "term_id": "GO:0031410"
}